limb epidermis development [GO:0060887] (biological process) Subtypes: limb epidermis stratification [GO:0060888] Relationships: is a type of GO:0098773; is part of limb development [GO:0060173] Sources: GOC:dph, GOC:sdb_2009, GOC:tb Definition: The process whose specific outcome is the progression of the epidermis of the limb over time, from its formation to the mature structure. The limb epidermis is the outer epithelial layer of the limb, it is a complex stratified squamous epithelium.